protein catabolic process in the vacuole [GO:0007039] (biological process) Also known as: vacuolar protein breakdown, vacuolar protein catabolic process, vacuolar protein catabolism, vacuolar protein degradation Regulation: regulated by regulation of protein catabolic process in the vacuole [GO:1904350]; negatively regulated by negative regulation of protein catabolic process in the vacuole [GO:1904351]; positively regulated by GO:1904352 Definition: The chemical reactions and pathways resulting in the breakdown of a protein in the vacuole, usually by the action of vacuolar proteases. Relationships: is a type of protein catabolic process [GO:0030163]; occurs in vacuole [GO:0005773] Sources: GOC:mah, GOC:vw Subtypes: GO:1905146